{
  "gene_symbol": "CLDN23",
  "term_id": "UNKNOWN:0001",
  "gene_name": "Claudin-23",
  "gene": "UniProtKB:Q96B33",
  "term_label": "Unknown molecular function"
}